{
  "term_id": "GO:0043235",
  "gene_symbol": "PRLR",
  "gene": "UniProtKB:P16471",
  "term_label": "receptor complex",
  "gene_name": "Prolactin receptor"
}